negative regulation of protein phosphorylation [GO:0001933] (biological process) Definition: Any process that stops, prevents or reduces the rate of addition of phosphate groups to amino acids within a protein. Also known as: down regulation of protein amino acid phosphorylation, down-regulation of protein amino acid phosphorylation, downregulation of protein amino acid phosphorylation, negative regulation of protein amino acid phosphorylation, inhibition of protein amino acid phosphorylation Subtypes: negative regulation of protein kinase activity [GO:0006469], negative regulation of peptidyl-threonine phosphorylation [GO:0010801], negative regulation of protein autophosphorylation [GO:0031953], GO:0033137, negative regulation of peptidyl-tyrosine phosphorylation [GO:0050732], GO:1903720, GO:1903912, GO:1904324 Relationships: is_a GO:0001932; is a type of negative regulation of protein modification process [GO:0031400]; is a type of negative regulation of phosphorylation [GO:0042326]; negatively regulates protein phosphorylation [GO:0006468] Sources: GOC:hjd